{
  "gene": "UniProtKB:Q9UPW8",
  "gene_symbol": "UNC13A",
  "gene_name": "Protein unc-13 homolog A",
  "term_id": "GO:0005886",
  "term_label": "plasma membrane"
}